lysine decarboxylase activity [GO:0008923] (molecular function) Sources: RHEA:22352 Also known as: L-lysine carboxy-lyase activity Relationships: is a type of carboxy-lyase activity [GO:0016831] Definition: Catalysis of the reaction: L-lysine + H+ = cadaverine + CO2.